{
  "term_label": "transcription regulator complex",
  "gene_name": "Neuronal PAS domain-containing protein 4",
  "gene_symbol": "NPAS4",
  "term_id": "GO:0005667",
  "gene": "UniProtKB:Q8IUM7"
}